{
  "gene_symbol": "CRLF1",
  "gene": "UniProtKB:O75462",
  "term_id": "GO:0043235",
  "term_label": "receptor complex",
  "gene_name": "Cytokine receptor-like factor 1"
}